{
  "gene": "UniProtKB:P15918",
  "gene_name": "V(D)J recombination-activating protein 1",
  "term_label": "ubiquitin protein ligase activity",
  "term_id": "GO:0061630",
  "gene_symbol": "RAG1"
}